cell body [GO:0044297] (CC) Definition: The portion of a cell bearing surface projections such as axons, dendrites, cilia, or flagella that includes the nucleus, but excludes all cell projections. Sources: GOC:go_curators Also known as: cell soma Note: Note that 'cell body' and 'cell soma' are not used in the literature for cells that lack projections, nor for some cells (e.g. yeast with mating projections) that do have projections. Relationships: is a type of cellular anatomical structure [GO:0110165] Subtypes: neuronal cell body [GO:0043025], somatic portion of tanycyte [GO:1990017]